{
  "gene_name": "Band 4.1-like protein 3",
  "gene_symbol": "EPB41L3",
  "gene": "UniProtKB:Q9Y2J2",
  "term_label": "cytoskeleton",
  "term_id": "GO:0005856"
}